{
  "gene_symbol": "CMC1",
  "gene_name": "COX assembly mitochondrial protein homolog",
  "term_id": "GO:0005739",
  "term_label": "mitochondrion",
  "gene": "UniProtKB:Q7Z7K0"
}